{
  "term_id": "GO:0003713",
  "gene_symbol": "DYRK1A",
  "gene": "UniProtKB:Q13627",
  "term_label": "transcription coactivator activity",
  "gene_name": "Dual specificity tyrosine-phosphorylation-regulated kinase 1A"
}